{
  "term_label": "Unknown molecular function",
  "gene": "UniProtKB:Q5JX71",
  "term_id": "UNKNOWN:0001",
  "gene_name": "Protein FAM209A",
  "gene_symbol": "FAM209A"
}